{
  "term_label": "calcitonin receptor binding",
  "gene_name": "Calcitonin",
  "gene": "UniProtKB:P01258",
  "term_id": "GO:0031716",
  "gene_symbol": "CALCA"
}